{
  "gene_name": "Sodium_hydrogen exchanger 4",
  "term_label": "sodium:proton antiporter activity",
  "gene_symbol": "SLC9A4",
  "term_id": "GO:0015385",
  "gene": "UniProtKB:Q6AI14"
}